{
  "gene_symbol": "CILP2",
  "term_label": "Unknown biological process",
  "gene": "UniProtKB:Q8IUL8",
  "term_id": "UNKNOWN:0002",
  "gene_name": "Cartilage intermediate layer protein 2"
}